DNA exonuclease activity, producing 5'-phosphomonoesters [GO:0016895] (molecular function) Also known as: exodeoxyribonuclease activity, producing 5' phosphomonoesters, exonuclease VIII activity Subtypes: 3'-5'-DNA exonuclease activity [GO:0008296], single-stranded DNA exodeoxyribonuclease activity [GO:0008297], GO:0008309, exodeoxyribonuclease V activity [GO:0008854], GO:0008855, 5'-3' DNA exonuclease activity [GO:0035312] Relationships: is a type of DNA exonuclease activity [GO:0004529] Definition: Catalysis of the hydrolysis of ester linkages within deoxyribonucleic acids by removing nucleotide residues from the 3' or 5' end to yield 5' phosphomonoesters. Sources: GOC:ai